{
  "gene": "UniProtKB:Q8IWB1",
  "gene_name": "Inositol 1,4,5-trisphosphate receptor-interacting protein",
  "gene_symbol": "ITPRIP",
  "term_id": "GO:0016020",
  "term_label": "membrane"
}